{
  "gene_symbol": "CHD8",
  "gene_name": "Chromodomain-helicase-DNA-binding protein 8",
  "term_id": "GO:0045892",
  "term_label": "negative regulation of DNA-templated transcription",
  "gene": "UniProtKB:Q9HCK8"
}